lateral inhibition [GO:0046331] (biological process) Definition: Signaling between cells of equivalent developmental potential that results in these cells adopting different developmental fates. An example is the suppression by cells with a particular fate of the adoption of the same fate by surrounding cells. Relationships: is a type of cell-cell signaling involved in cell fate commitment [GO:0045168] Sources: GOC:bf, GOC:kmv